{
  "term_label": "plasma membrane",
  "gene": "UniProtKB:Q8IU80",
  "gene_symbol": "TMPRSS6",
  "gene_name": "Transmembrane protease serine 6",
  "term_id": "GO:0005886"
}